{
  "term_id": "GO:0045947",
  "gene_symbol": "GIGYF1",
  "gene": "UniProtKB:O75420",
  "gene_name": "GRB10-interacting GYF protein 1",
  "term_label": "negative regulation of translational initiation"
}